{
  "term_id": "GO:0005737",
  "gene_name": "Ubiquitin thioesterase otulin",
  "gene_symbol": "OTULIN",
  "term_label": "cytoplasm",
  "gene": "UniProtKB:Q96BN8"
}